{
  "gene": "UniProtKB:A6NLP5",
  "gene_symbol": "TTC36",
  "gene_name": "Tetratricopeptide repeat protein 36",
  "term_label": "Unknown cellular component",
  "term_id": "UNKNOWN:0003"
}